{
  "term_id": "GO:0051967",
  "gene_name": "D(3) dopamine receptor",
  "term_label": "negative regulation of synaptic transmission, glutamatergic",
  "gene": "UniProtKB:P35462",
  "gene_symbol": "DRD3"
}